{
  "gene_name": "Calcium_calmodulin-dependent protein kinase type II subunit beta",
  "gene_symbol": "CAMK2B",
  "term_id": "GO:0005516",
  "term_label": "calmodulin binding",
  "gene": "UniProtKB:Q13554"
}